{
  "term_id": "GO:0005743",
  "gene_symbol": "CYP11B1",
  "gene": "UniProtKB:P15538",
  "term_label": "mitochondrial inner membrane",
  "gene_name": "Cytochrome P450 11B1, mitochondrial"
}